N-acetylglucosamine deacetylase activity [GO:0050119] (molecular function) Sources: EC:3.5.1.33, RHEA:20593 Definition: Catalysis of the reaction: N-acetyl-D-glucosamine + H2O = D-glucosamine + acetate. Relationships: is a type of hydrolase activity, acting on carbon-nitrogen (but not peptide) bonds, in linear amides [GO:0016811]; is a type of deacetylase activity [GO:0019213] Also known as: N-acetyl-D-glucosamine amidohydrolase activity, N-acetyl-D-glucosaminyl N-deacetylase activity, acetylaminodeoxyglucose acetylhydrolase activity